{
  "gene": "UniProtKB:Q9H4L7",
  "gene_name": "SWI_SNF-related matrix-associated actin-dependent regulator of chromatin subfamily A containing DEAD_H box 1",
  "term_label": "nucleosome array spacer activity",
  "gene_symbol": "SMARCAD1",
  "term_id": "GO:0140750"
}